2-furoyl-CoA dehydrogenase activity [GO:0047542] (molecular function) Also known as: 2-furoyl coenzyme A dehydrogenase activity, 2-furoyl coenzyme A hydroxylase activity, 2-furoyl-CoA:(acceptor) 5-oxidoreductase (hydroxylating), 2-furoyl-CoA:acceptor 5-oxidoreductase (hydroxylating), furoyl-CoA hydroxylase activity Relationships: is a type of oxidoreductase activity, acting on the CH-CH group of donors [GO:0016627] Definition: Catalysis of the reaction: 2-furoyl-CoA + A + H2O = 5-hydroxy-2-furoyl-CoA + AH(2) + H+. Sources: EC:1.3.99.8, RHEA:21480